{
  "term_label": "opioid receptor binding",
  "gene_name": "Proenkephalin-B",
  "gene": "UniProtKB:P01213",
  "gene_symbol": "PDYN",
  "term_id": "GO:0031628"
}